{
  "term_id": "GO:0005634",
  "gene_name": "Putative zinc finger protein 137",
  "term_label": "nucleus",
  "gene": "UniProtKB:P52743",
  "gene_symbol": "ZNF137P"
}